symbiont-mediated perturbation of host actin cytoskeleton via actin filament reorganization [GO:0141032] (biological process) Also known as: perturbation by symbiont of host actin cytoskeleton via actin filament rearrangement, perturbation by symbiont of host actin cytoskeleton via actin filament reorganization Relationships: is a type of symbiont-mediated perturbation of host actin cytoskeleton [GO:0141027] References: PMID:22212282, PMID:31130928 Definition: The process in which an organism effects a change that impairs the structure or function of the host actin cytoskeleton by reorganizing the actin filaments, in a way that keeps the total filementous actin remains approximately constant. The host is defined as the larger of the organisms involved in a symbiotic interaction.